heme receptor activity [GO:0140488] (molecular function) References: PMID:28193844, PMID:32185489 Definition: Binding specifically to heme to deliver it to a transport vesicle. Relationships: is a type of cargo receptor activity [GO:0038024]